{
  "term_label": "cyclin-dependent protein kinase holoenzyme complex",
  "gene_name": "Cyclin-dependent kinase 16",
  "gene_symbol": "CDK16",
  "term_id": "GO:0000307",
  "gene": "UniProtKB:Q00536"
}